{
  "gene_symbol": "TMEM72",
  "gene_name": "Transmembrane protein 72",
  "term_id": "UNKNOWN:0003",
  "gene": "UniProtKB:A0PK05",
  "term_label": "Unknown cellular component"
}